(+)-abscisic acid 8'-hydroxylase activity [GO:0010295] (molecular function) Definition: Catalysis of the reaction: (+)-abscisate + H+ + NADPH + O2 = (+)-8'-hydroxyabscisate + H2O + NADP+. Also known as: abscisic acid 8'-hydroxylase activity, (+)-ABA 8'-hydroxylase activity, ABA 8'-Hydroxylase activity, Abscisate 8'-hydroxylase activity, ABA 8'-hydroxylase activity, abscisate,NADPH:oxygen oxidoreductase (8'-hydroxylating) Sources: EC:1.14.14.137, RHEA:12897 Relationships: is_a oxidoreductase activity, acting on paired donors, with incorporation or reduction of molecular oxygen, NAD(P)H as one donor, and incorporation of one atom of oxygen [GO:0016709]